{
  "term_id": "GO:0007368",
  "gene_symbol": "NEK8",
  "gene": "UniProtKB:Q86SG6",
  "gene_name": "Serine_threonine-protein kinase Nek8",
  "term_label": "determination of left/right symmetry"
}